{
  "gene_name": "Histone RNA hairpin-binding protein",
  "gene_symbol": "SLBP",
  "term_id": "GO:0071207",
  "gene": "UniProtKB:Q14493",
  "term_label": "histone pre-mRNA stem-loop binding"
}